{
  "gene_symbol": "IHH",
  "gene_name": "Indian hedgehog protein",
  "gene": "UniProtKB:Q14623",
  "term_label": "patched binding",
  "term_id": "GO:0005113"
}